{
  "term_label": "odorant binding",
  "gene_symbol": "OR5A2",
  "gene": "UniProtKB:Q8NGI9",
  "term_id": "GO:0005549",
  "gene_name": "Olfactory receptor 5A2"
}